{
  "gene": "UniProtKB:Q8NGC8",
  "term_label": "Unknown molecular function",
  "gene_symbol": "OR11H7",
  "term_id": "UNKNOWN:0001",
  "gene_name": "Olfactory receptor 11H7"
}